{
  "term_label": "Unknown cellular component",
  "term_id": "UNKNOWN:0003",
  "gene": "UniProtKB:Q8NDV2",
  "gene_name": "G-protein coupled receptor 26",
  "gene_symbol": "GPR26"
}